{
  "gene_symbol": "VPS33B",
  "term_id": "GO:0033263",
  "gene": "UniProtKB:Q9H267",
  "term_label": "CORVET complex",
  "gene_name": "Vacuolar protein sorting-associated protein 33B"
}